{
  "term_label": "G protein-coupled serotonin receptor activity",
  "term_id": "GO:0004993",
  "gene_symbol": "HTR2C",
  "gene_name": "5-hydroxytryptamine receptor 2C",
  "gene": "UniProtKB:P28335"
}